ATP-dependent DNA/DNA annealing activity [GO:0036310] (molecular function) Relationships: is a type of ATP-dependent activity, acting on DNA [GO:0008094]; is a type of DNA/DNA annealing activity [GO:1990814] References: PMID:21078962, PMID:22704558, PMID:22705370, PMID:22759634, PMID:22888405 Also known as: nucleoside-triphosphatase activity involved in DNA annealing, ATP-dependent DNA annealing activity, DNA rewinding activity, annealing helicase activity Definition: An ATP-dependent activity that facilitates the formation of a complementary double-stranded DNA molecule.